germline cell cycle switching, mitotic to meiotic cell cycle [GO:0051729] (biological process) Sources: GOC:ai Definition: The process in which a germline cell switches cell cycle mode from mitotic to meiotic division. Relationships: is a type of cell cycle switching, mitotic to meiotic cell cycle [GO:0051728] Also known as: germline conversion to meiotic cell cycle, germline entry into meiotic cell cycle, germline initiation of meiotic cell cycle, germline cell cycle switching, mitosis to meiosis, germline conversion to meiosis, germline entry into meiosis, germline initiation of meiosis, germline meiotic entry